mitotic spindle microtubule [GO:1990498] (cellular component) Definition: Any microtubule that is part of a mitotic spindle; anchored at one spindle pole. Subtypes: mitotic spindle polar microtubule [GO:1990537], mitotic spindle kinetochore microtubule [GO:1990941] Sources: GOC:vw Relationships: is a type of spindle microtubule [GO:0005876]; is part of GO:0072686